{
  "gene_name": "T-cell surface glycoprotein CD3 gamma chain",
  "term_label": "alpha-beta T cell receptor complex",
  "gene_symbol": "CD3G",
  "gene": "UniProtKB:P09693",
  "term_id": "GO:0042105"
}